{
  "gene_name": "Chondrosarcoma-associated gene 1 protein",
  "term_id": "UNKNOWN:0002",
  "gene": "UniProtKB:Q6PB30",
  "gene_symbol": "CSAG1",
  "term_label": "Unknown biological process"
}